{
  "gene": "UniProtKB:Q8WW35",
  "term_id": "GO:0005737",
  "term_label": "cytoplasm",
  "gene_name": "Dynein light chain Tctex-type protein 2B",
  "gene_symbol": "DYNLT2B"
}